{
  "term_label": "DNA-binding transcription factor activity, RNA polymerase II-specific",
  "gene_name": "Krueppel-like factor 12",
  "gene": "UniProtKB:Q9Y4X4",
  "gene_symbol": "KLF12",
  "term_id": "GO:0000981"
}